{
  "term_id": "GO:0019901",
  "gene_symbol": "RHOG",
  "term_label": "protein kinase binding",
  "gene_name": "Rho-related GTP-binding protein RhoG",
  "gene": "UniProtKB:P84095"
}